positive regulation of protein secretion [GO:0050714] (BP) Subtypes: positive regulation of insulin secretion [GO:0032024], positive regulation of Wnt protein secretion [GO:0061357], GO:0070165, GO:0090340, positive regulation of renin secretion into blood stream [GO:1900135], positive regulation of BMP secretion [GO:1900144], GO:1902278, positive regulation of prolactin secretion [GO:1902722], positive regulation of pancreatic trypsinogen secretion [GO:1904244], positive regulation of matrix metallopeptidase secretion [GO:1904466] Sources: GOC:ai Definition: Any process that activates or increases the frequency, rate or extent of the controlled release of a protein from a cell. Also known as: up regulation of protein secretion, up-regulation of protein secretion, upregulation of protein secretion, activation of protein secretion, stimulation of protein secretion Relationships: is a type of GO:0050708; is a type of GO:0051222; is a type of positive regulation of secretion by cell [GO:1903532]; positively regulates protein secretion [GO:0009306]